negative regulation of Schwann cell chemotaxis [GO:1904267] (BP) References: PMID:16203995 Sources: GOC:TermGenie, GO_REF:0000058 Relationships: is a type of negative regulation of chemotaxis [GO:0050922]; is a type of GO:1900148; is a type of GO:1904266; negatively regulates Schwann cell chemotaxis [GO:1990751] Also known as: down regulation of Schwann cell chemotaxis, down-regulation of Schwann cell chemotaxis, downregulation of Schwann cell chemotaxis, inhibition of Schwann cell chemotaxis Definition: Any process that stops, prevents or reduces the frequency, rate or extent of Schwann cell chemotaxis.